negative regulation of antifungal peptide production [GO:0002789] (biological process) Relationships: is a type of negative regulation of antimicrobial peptide production [GO:0002785]; is a type of GO:0002788; negatively regulates antifungal peptide production [GO:0002781] Sources: GOC:add Definition: Any process that stops, prevents, or reduces the frequency, rate, or extent of antifungal peptide production. Subtypes: negative regulation of antifungal peptide secretion [GO:0002801], GO:0002811 Also known as: down regulation of antifungal peptide production, down-regulation of antifungal peptide production, downregulation of antifungal peptide production, inhibition of antifungal peptide production